{
  "term_label": "mitochondrial inner membrane",
  "gene_symbol": "CYP11B2",
  "gene": "UniProtKB:P19099",
  "gene_name": "Cytochrome P450 11B2, mitochondrial",
  "term_id": "GO:0005743"
}